{
  "gene_symbol": "ALKBH8",
  "gene": "UniProtKB:Q96BT7",
  "gene_name": "Alkylated DNA repair protein alkB homolog 8",
  "term_id": "GO:0106335",
  "term_label": "tRNA (5-carboxymethyluridine(34)-5-O)-methyltransferase activity"
}